{
  "term_id": "GO:0005634",
  "gene_name": "Pseudouridylate synthase 1 homolog",
  "gene_symbol": "PUS1",
  "gene": "UniProtKB:Q9Y606",
  "term_label": "nucleus"
}